{
  "gene_name": "Glypican-6",
  "gene": "UniProtKB:Q9Y625",
  "term_label": "regulation of neurotransmitter receptor localization to postsynaptic specialization membrane",
  "gene_symbol": "GPC6",
  "term_id": "GO:0098696"
}